{
  "gene_name": "Cytosolic arginine sensor for mTORC1 subunit 2",
  "gene": "UniProtKB:A6NHX0",
  "gene_symbol": "CASTOR2",
  "term_id": "GO:1904262",
  "term_label": "negative regulation of TORC1 signaling"
}